{
  "term_id": "GO:0004674",
  "term_label": "protein serine/threonine kinase activity",
  "gene_symbol": "STK39",
  "gene": "UniProtKB:Q9UEW8",
  "gene_name": "STE20_SPS1-related proline-alanine-rich protein kinase"
}